{
  "term_label": "extracellular space",
  "term_id": "GO:0005615",
  "gene_name": "Tenascin-X",
  "gene_symbol": "TNXB",
  "gene": "UniProtKB:P22105"
}